dorsal closure, leading edge cell fate determination [GO:0007393] (BP) Relationships: is a type of leading edge cell fate determination [GO:0035028]; is part of dorsal closure, leading edge cell fate commitment [GO:0035029] Definition: The cell fate determination process in which a cell within the dorsal ectoderm becomes capable of differentiating autonomously into a leading edge cell regardless of its environment; upon determination, the cell fate cannot be reversed. References: PMID:12147138 Sources: GOC:bf, GOC:go_curators